{
  "gene_symbol": "CDK5RAP2",
  "gene_name": "CDK5 regulatory subunit-associated protein 2",
  "gene": "UniProtKB:Q96SN8",
  "term_label": "mitotic spindle pole",
  "term_id": "GO:0097431"
}